{
  "gene_name": "cTAGE family member 8",
  "term_id": "UNKNOWN:0001",
  "gene": "UniProtKB:P0CG41",
  "term_label": "Unknown molecular function",
  "gene_symbol": "CTAGE8"
}